histone H2AXS139 phosphatase activity [GO:0140791] (molecular function) Also known as: histone H2-S140 serine phosphatase activity, histone serine phosphatase activity (H2-S140 specific), histone H2S140 phosphatase activity References: PMID:18614045 Note: Note that the residue position corresponds to the canonical human H2AX histone (UniProtKB:P16104); this residue is conserved across all eukaryotes. Residue 1 is the first residue following removal of the initiating Methionine (Met). Note that each histone is encoded by multiple genes, and sequences may vary across different genes within an organism. Definition: Catalysis of the reaction: histone H2AX serine phosphate (position 139) + H2O = histone H2AX serine (position 139) + phosphate. Relationships: is a type of histone phosphatase activity [GO:0140789]